{
  "term_id": "GO:0016324",
  "gene_symbol": "SLC5A1",
  "gene": "UniProtKB:P13866",
  "gene_name": "Sodium_glucose cotransporter 1",
  "term_label": "apical plasma membrane"
}